establishment of latency as a linear episome [GO:0075530] (biological process) Relationships: is_a establishment of episomal latency [GO:0075720] Definition: A process by which a virus establishes a latent state within its host as an episome, where the viral genome remains silent in the cytoplasm or nucleus as linear structure. Sources: GOC:jl Also known as: establishment of latency as a linear plasmid, establishment of linear plasmid latency